dorsal spinal cord development [GO:0021516] (biological process) References: PMID:11179871 Sources: GOC:cls, GOC:dgh, GOC:dph, GOC:jid, GO_REF:0000021 Definition: The process whose specific outcome is the progression of the dorsal region of the spinal cord over time, from its formation to the mature structure. The dorsal region of the mature spinal cord contains neurons that process and relay sensory input. Relationships: is a type of anatomical structure development [GO:0048856]; is part of GO:0021510